phosphothreonine lyase activity [GO:0034598] (molecular function) References: PMID:17303758, PMID:18084305 Definition: Catalysis of the removal of the phosphate group from phosphothreonine by cleavage of the C-OP bond with the concomitant abstraction of the alpha proton, generating a double bond-containing product. Relationships: is a type of carbon-oxygen lyase activity, acting on phosphates [GO:0016838]